cellular localization [GO:0051641] (biological process) Note: Note that this term is in the subset of terms that should not be used for direct gene product annotation. Instead, select a child term or, if no appropriate child term exists, please request a new term. Direct annotations to this term may be amended during annotation QC. Also known as: cellular localisation, establishment and maintenance of cellular localization, establishment and maintenance of localization in cell or cell membrane, single organism cellular localization, intracellular localization, localization within cell, single-organism cellular localization Relationships: is a type of cellular process [GO:0009987]; is a type of localization [GO:0051179] Subtypes: intracellular transport [GO:0046907], actin cortical patch localization [GO:0051666], localization within membrane [GO:0051668], spindle pole body localization [GO:0070631], ribonucleoprotein complex localization [GO:0071166], stalled replication fork localization to nuclear periphery [GO:0120290] Regulation: regulated by regulation of cellular localization [GO:0060341] Definition: A cellular localization process whereby a substance or cellular entity, such as a protein complex or organelle, is transported to, and/or maintained in, a specific location within a cell including the localization of substances or cellular entities to the cell membrane. Sources: GOC:tb, GOC:vw